ISG15 conjugating enzyme activity [GO:0061653] (molecular function) Relationships: is a type of ISG15 transferase activity [GO:0042296]; is a type of ubiquitin-like protein conjugating enzyme activity [GO:0061650] Sources: GOC:dph Definition: Isoenergetic transfer of ISG15 from one protein to another via the reaction X-ISG15 + Y = Y-ISG15 + X, where both the X-ISG15 and Y-ISG15 linkages are thioester bonds between the C-terminal amino acid of ISG15 and a sulfhydryl side group of a cysteine residue. Also known as: E2